{
  "gene_name": "TGF-beta receptor type-2",
  "gene_symbol": "TGFBR2",
  "term_id": "GO:0032924",
  "term_label": "activin receptor signaling pathway",
  "gene": "UniProtKB:P37173"
}